{
  "term_label": "Unknown molecular function",
  "term_id": "UNKNOWN:0001",
  "gene_name": "Protein FMC1 homolog",
  "gene_symbol": "FMC1",
  "gene": "UniProtKB:Q96HJ9"
}